{
  "term_label": "olfactory receptor activity",
  "term_id": "GO:0004984",
  "gene_name": "Olfactory receptor 2W1",
  "gene": "UniProtKB:Q9Y3N9",
  "gene_symbol": "OR2W1"
}